{
  "term_id": "UNKNOWN:0002",
  "gene_symbol": "KRTAP10-11",
  "gene": "UniProtKB:P60412",
  "term_label": "Unknown biological process",
  "gene_name": "Keratin-associated protein 10-11"
}